{
  "term_label": "microtubule cytoskeleton",
  "gene": "UniProtKB:Q8IYM1",
  "term_id": "GO:0015630",
  "gene_name": "Septin-12",
  "gene_symbol": "SEPTIN12"
}